{
  "term_id": "GO:0005886",
  "gene": "UniProtKB:B9EJG8",
  "gene_name": "Transmembrane protein 150C",
  "term_label": "plasma membrane",
  "gene_symbol": "TMEM150C"
}